glucuronate catabolic process [GO:0006064] (biological process) Definition: The chemical reactions and pathways resulting in the breakdown of glucuronate, any salt or ester of glucuronic acid. Also known as: glucuronate breakdown, glucuronate catabolism, glucuronate degradation Sources: GOC:go_curators Relationships: is_a GO:0019585; is a type of monocarboxylic acid catabolic process [GO:0072329] Subtypes: D-glucuronate catabolic process [GO:0042840]